(S)-nandinine synthase activity [GO:0102632] (molecular function) Definition: Catalysis of the reaction: (S)-scoulerine + reduced [NADPH--hemoprotein reductase] + O2 = (S)-nandinine + oxidized [NADPH--hemoprotein reductase] + 2 H2O + H+. Relationships: is a type of oxidoreductase activity, acting on paired donors, with oxidation of a pair of donors resulting in the reduction of molecular oxygen to two molecules of water [GO:0016717] References: PMID:17250743, PMID:21094631 Sources: RHEA:50364